{
  "gene_name": "Checkpoint protein HUS1",
  "gene_symbol": "HUS1",
  "gene": "UniProtKB:O60921",
  "term_id": "GO:0030896",
  "term_label": "checkpoint clamp complex"
}